{
  "gene": "UniProtKB:Q9UJ99",
  "term_id": "GO:0016342",
  "gene_symbol": "CDH22",
  "gene_name": "Cadherin-22",
  "term_label": "catenin complex"
}